{
  "term_id": "GO:0004476",
  "gene_name": "Mannose-6-phosphate isomerase",
  "gene_symbol": "MPI",
  "term_label": "mannose-6-phosphate isomerase activity",
  "gene": "UniProtKB:P34949"
}